dihydrocoumarin hydrolase activity [GO:0047856] (molecular function) Sources: RHEA:10360 Also known as: 3,4-dihydrocoumarin hydrolase activity, dihydrocoumarin lipase activity, dihydrocoumarin lactonohydrolase activity Relationships: is a type of carboxylic ester hydrolase activity [GO:0052689] Definition: Catalysis of the reaction: 3,4-dihydrocoumarin + H2O = 3-(2-hydroxyphenyl)propanoate + H+.